venous endothelial cell migration involved in lymph vessel development [GO:0060855] (biological process) Definition: The orderly movement of venous endothelial cells out of the veins giving rise to the precursors of lymphatic endothelial cells. Relationships: is a type of blood vessel endothelial cell migration [GO:0043534]; is part of lymph vessel development [GO:0001945] Sources: GOC:dph, GOC:sdb_2009, GOC:tb